carbon monoxide binding [GO:0070025] (molecular function) Relationships: is a type of small molecule binding [GO:0036094] Sources: GOC:ecd Also known as: CO binding Definition: Binding to carbon monoxide (CO).